{
  "gene": "UniProtKB:Q9H7Z3",
  "term_label": "negative regulation of RNA catabolic process",
  "gene_name": "Nuclear exosome regulator NRDE2",
  "term_id": "GO:1902369",
  "gene_symbol": "NRDE2"
}